{
  "gene": "UniProtKB:P07948",
  "gene_name": "Tyrosine-protein kinase Lyn",
  "gene_symbol": "LYN",
  "term_id": "GO:0004715",
  "term_label": "non-membrane spanning protein tyrosine kinase activity"
}